{
  "gene": "UniProtKB:Q99865",
  "term_label": "cytosol",
  "gene_name": "Spindlin-2A",
  "term_id": "GO:0005829",
  "gene_symbol": "SPIN2A"
}